{
  "term_label": "carbohydrate binding",
  "gene_name": "C-type lectin domain family 4 member F",
  "term_id": "GO:0030246",
  "gene": "UniProtKB:Q8N1N0",
  "gene_symbol": "CLEC4F"
}